{
  "gene_symbol": "MAOB",
  "term_label": "phenylethylamine catabolic process",
  "gene": "UniProtKB:P27338",
  "term_id": "GO:0019607",
  "gene_name": "Amine oxidase [flavin-containing] B"
}